{
  "term_id": "GO:0000795",
  "gene_name": "Synaptonemal complex protein 3",
  "gene_symbol": "SYCP3",
  "gene": "UniProtKB:Q8IZU3",
  "term_label": "synaptonemal complex"
}